sodium ion-transporting two-sector ATPase complex [GO:0016472] (cellular component) Relationships: is a type of membrane protein complex [GO:0098796] Definition: A large protein complex that catalyzes the synthesis or hydrolysis of ATP by a rotational mechanism, coupled to the transport of sodium ions across a membrane. The complex comprises a membrane sector (F0 or V0) that carries out ion transport and a cytoplasmic compartment sector (F1 or V1) that catalyzes ATP synthesis or hydrolysis. Also known as: sodium-transporting two-sector ATPase complex References: PMID:14656431 Sources: GOC:mah Subtypes: sodium ion-transporting F-type ATPase complex [GO:0016473], sodium ion-transporting V-type ATPase complex [GO:0016474]